{
  "gene": "UniProtKB:Q8IWX7",
  "gene_name": "Protein unc-45 homolog B",
  "term_label": "Hsp90 protein binding",
  "term_id": "GO:0051879",
  "gene_symbol": "UNC45B"
}